{
  "term_id": "GO:0034341",
  "gene_name": "Putative dispanin subfamily A member 2d",
  "term_label": "response to type II interferon",
  "gene_symbol": "C9JQL5",
  "gene": "UniProtKB:C9JQL5"
}